protein phosphatase inhibitor complex [GO:0062049] (cellular component) References: PMID:19407142, PMID:19933100 Sources: GOC:bhm Definition: A protein-containing complex that inhibits protein phosphatase activity by directly binding to a protein phosphatase. Relationships: is a type of GO:0032991